regulation of adiponectin secretion [GO:0070163] (biological process) Sources: GOC:mah Subtypes: negative regulation of adiponectin secretion [GO:0070164], positive regulation of adiponectin secretion [GO:0070165] Definition: Any process that modulates the frequency, rate or extent of the regulated release of adiponectin from a cell. Relationships: is a type of regulation of hormone secretion [GO:0046883]; is_a regulation of protein secretion [GO:0050708]; regulates adiponectin secretion [GO:0070162]